{
  "gene_name": "Protein EVI2B",
  "gene": "UniProtKB:P34910",
  "term_label": "regulation of stem cell division",
  "term_id": "GO:2000035",
  "gene_symbol": "EVI2B"
}